phagosome-lysosome fusion [GO:0090385] (biological process) Relationships: is a type of vesicle fusion [GO:0006906]; is part of phagolysosome assembly [GO:0001845] Sources: GOC:kmv, GOC:tb Subtypes: GO:0090389 Definition: The creation of a phagolysosome from a phagosome and a lysosome.